{
  "gene_symbol": "FPR2",
  "gene": "UniProtKB:P25090",
  "term_id": "GO:0007200",
  "term_label": "phospholipase C-activating G protein-coupled receptor signaling pathway",
  "gene_name": "N-formyl peptide receptor 2"
}